{
  "gene": "UniProtKB:Q2TBE0",
  "term_id": "GO:0071014",
  "gene_name": "CWF19-like protein 2",
  "gene_symbol": "CWF19L2",
  "term_label": "post-mRNA release spliceosomal complex"
}